{
  "gene_name": "Trafficking protein particle complex subunit 14",
  "gene": "UniProtKB:Q8WVR3",
  "term_id": "GO:1990071",
  "gene_symbol": "TRAPPC14",
  "term_label": "TRAPPII protein complex"
}